regulatory RNA binding [GO:0061980] (molecular function) Definition: Binding to a small regulatory RNA, a short RNA (usually 50-200 nt long) that is either independently transcribed or processed from a longer RNA by an RNAse enzyme. References: PMID:14622403, PMID:23475961 Relationships: is a type of RNA binding [GO:0003723] Subtypes: GO:0034584, GO:0035197, miRNA binding [GO:0035198]